{
  "gene_symbol": "FRMD4B",
  "term_id": "UNKNOWN:0002",
  "gene_name": "FERM domain-containing protein 4B",
  "gene": "UniProtKB:Q9Y2L6",
  "term_label": "Unknown biological process"
}